{
  "gene_name": "26S proteasome non-ATPase regulatory subunit 13",
  "term_id": "GO:0008541",
  "term_label": "proteasome regulatory particle, lid subcomplex",
  "gene_symbol": "PSMD13",
  "gene": "UniProtKB:Q9UNM6"
}